{
  "gene_name": "Serpin B9",
  "term_label": "cytoplasm",
  "gene_symbol": "SERPINB9",
  "term_id": "GO:0005737",
  "gene": "UniProtKB:P50453"
}